{
  "gene": "UniProtKB:Q8WTU0",
  "gene_name": "Protein DDI1 homolog 1",
  "gene_symbol": "DDI1",
  "term_label": "proteasomal protein catabolic process",
  "term_id": "GO:0010498"
}